cell proliferation involved in heart morphogenesis [GO:0061323] (biological process) Definition: The multiplication or reproduction of cells, resulting in the expansion of a cell population that contributes to the shaping of the heart. Sources: GOC:dph, GOC:mtg_heart Relationships: is a type of cell population proliferation [GO:0008283]; is part of heart morphogenesis [GO:0003007] Subtypes: cell proliferation involved in heart valve morphogenesis [GO:0003249], GO:0003263, cell proliferation involved in atrial ventricular junction remodeling [GO:0003295], GO:0061325, fibroblast proliferation involved in heart morphogenesis [GO:0061385], GO:1905315 Regulation: regulated by regulation of cell proliferation involved in heart morphogenesis [GO:2000136]; negatively regulated by negative regulation of cell proliferation involved in heart morphogenesis [GO:2000137]; positively regulated by positive regulation of cell proliferation involved in heart morphogenesis [GO:2000138]